{
  "term_id": "GO:0001916",
  "term_label": "positive regulation of T cell mediated cytotoxicity",
  "gene": "UniProtKB:P29016",
  "gene_symbol": "CD1B",
  "gene_name": "T-cell surface glycoprotein CD1b"
}